regulation of methyl-branched fatty acid biosynthetic process [GO:1902322] (biological process) Subtypes: negative regulation of methyl-branched fatty acid biosynthetic process [GO:1902323], GO:1902324 Also known as: regulation of methyl-branched fatty acid anabolism, regulation of methyl-branched fatty acid biosynthesis, regulation of methyl-branched fatty acid formation, regulation of methyl-branched fatty acid synthesis Definition: Any process that modulates the frequency, rate or extent of methyl-branched fatty acid biosynthetic process. References: PMID:15340492 Sources: GOC:TermGenie, GOC:kmv Relationships: is a type of regulation of fatty acid biosynthetic process [GO:0042304]; regulates methyl-branched fatty acid biosynthetic process [GO:1902321]